positive regulation of border follicle cell migration [GO:1903688] (biological process) Definition: Any process that activates or increases the frequency, rate or extent of border follicle cell migration. References: PMID:18394891 Sources: GOC:TermGenie, GOC:als, GO_REF:0000058 Also known as: activation of border follicle cell migration Relationships: is a type of positive regulation of epithelial cell migration [GO:0010634]; is a type of regulation of border follicle cell migration [GO:1903684]; positively regulates border follicle cell migration [GO:0007298]